{
  "term_id": "GO:0005737",
  "gene_name": "Prefoldin subunit 3",
  "gene_symbol": "VBP1",
  "term_label": "cytoplasm",
  "gene": "UniProtKB:P61758"
}